RNAi-mediated antiviral immune response [GO:0009616] (biological process) Definition: A post-transcriptional gene silencing pathway mediated by the action of regulatory RNAs that protects against foreign organism invasion by restricting viral replication and dissemination. Note: Virus induced gene silencing (VIGS) is used as a technique to control plant gene expression; when used in that context, this does not represent a normal biological process and is outside the scope of GO. Also known as: RNAi-mediated antiviral immunity, virus induced gene silencing, virus-induced PTGS, virus-induced gene silencing, VIGS, viral gene silencing in virus induced gene silencing, viral triggering of virus induced gene silencing Subtypes: GO:0051214, RNAi-mediated antiviral immunity against DNA virus [GO:0051215] Relationships: is a type of GO:0035194; is a type of innate immune response [GO:0045087]; is a type of GO:0051607 References: PMID:17693253, PMID:21724934, PMID:23686236, PMID:24732439, PMID:31100912 Sources: GOC:jl